deoxynucleoside phosphate kinase activity, dGTP as phosphate donor [GO:0106367] (molecular function) References: PMID:20497505 Sources: RHEA:62128 Definition: Catalysis of the reaction: a 2'-deoxyribonucleoside 5'-phosphate + dGTP = a 2'-deoxyribonucleoside 5'-diphosphate + dGDP. Relationships: is a type of GO:0016776; is a type of GO:0019205